{
  "gene": "UniProtKB:O95721",
  "gene_symbol": "SNAP29",
  "gene_name": "Synaptosomal-associated protein 29",
  "term_label": "SNARE complex",
  "term_id": "GO:0031201"
}